{
  "gene": "UniProtKB:Q9H6F2",
  "gene_name": "Trimeric intracellular cation channel type A",
  "term_label": "potassium ion transmembrane transport",
  "term_id": "GO:0071805",
  "gene_symbol": "TMEM38A"
}